UDP-N-acetyl-D-mannosamine dehydrogenase activity [GO:0089714] (molecular function) Sources: EC:1.1.1.336 Relationships: is_a oxidoreductase activity, acting on the CH-OH group of donors, NAD or NADP as acceptor [GO:0016616] Definition: Catalysis of the reaction: UDP-N-acetyl-alpha-D-mannosamine + 2 NAD+ + H2O = UDP-N-acetyl-alpha-D-mannosaminuronate + 2 NADH + 2 H+.